{
  "gene_name": "MORN repeat-containing protein 1",
  "term_label": "Unknown molecular function",
  "gene": "UniProtKB:Q5T089",
  "gene_symbol": "MORN1",
  "term_id": "UNKNOWN:0001"
}